establishment of neuroblast polarity [GO:0045200] (biological process) Definition: The specification and formation of the apicobasal polarity of a neuroblast cell, a progenitor of the central nervous system. Sources: GOC:bf, GOC:mtg_sensu Relationships: is a type of establishment of cell polarity [GO:0030010]; is a type of establishment or maintenance of neuroblast polarity [GO:0045196] Also known as: establishment of neuroblast cell polarity